negative regulation of signal transduction involved in conjugation with cellular fusion [GO:0060240] (biological process) Definition: Any process that decreases the rate, frequency or extent of the series signal transduction involved in conjugation with cellular fusion. Relationships: is a type of GO:0009968; is a type of regulation of signal transduction involved in conjugation with cellular fusion [GO:0060238]; is a type of negative regulation of reproductive process [GO:2000242]; negatively regulates GO:0032005 Subtypes: GO:0090029 Sources: GOC:dph, GOC:tb